{
  "term_id": "GO:0006508",
  "gene_symbol": "ADAM7",
  "gene": "UniProtKB:Q9H2U9",
  "gene_name": "Disintegrin and metalloproteinase domain-containing protein 7",
  "term_label": "proteolysis"
}